{
  "gene_symbol": "GPSM2",
  "term_id": "GO:0001965",
  "gene": "UniProtKB:P81274",
  "gene_name": "G-protein-signaling modulator 2",
  "term_label": "G-protein alpha-subunit binding"
}